{
  "gene": "UniProtKB:P57729",
  "term_label": "GTPase activity",
  "gene_symbol": "RAB38",
  "term_id": "GO:0003924",
  "gene_name": "Ras-related protein Rab-38"
}